{
  "gene_name": "Zinc finger protein 3 homolog",
  "gene": "UniProtKB:Q96NJ6",
  "term_label": "RNA polymerase II transcription regulatory region sequence-specific DNA binding",
  "term_id": "GO:0000977",
  "gene_symbol": "ZFP3"
}